{
  "gene": "UniProtKB:Q2NKQ1",
  "term_label": "GTPase activator activity",
  "term_id": "GO:0005096",
  "gene_name": "Small G protein signaling modulator 1",
  "gene_symbol": "SGSM1"
}